{
  "gene": "UniProtKB:P0CG43",
  "term_id": "UNKNOWN:0002",
  "gene_name": "Putative protein FAM157C",
  "gene_symbol": "FAM157C",
  "term_label": "Unknown biological process"
}